{
  "term_id": "GO:0005813",
  "term_label": "centrosome",
  "gene": "UniProtKB:O43303",
  "gene_name": "Centriolar coiled-coil protein of 110 kDa",
  "gene_symbol": "CCP110"
}